negative regulation of gamma-aminobutyric acid catabolic process [GO:1901716] (biological process) Definition: Any process that stops, prevents or reduces the frequency, rate or extent of gamma-aminobutyric acid catabolic process. Sources: GOC:TermGenie Relationships: is_a negative regulation of catabolic process [GO:0009895]; is a type of GO:0045763; is a type of negative regulation of small molecule metabolic process [GO:0062014]; is a type of GO:1901715; negatively regulates gamma-aminobutyric acid catabolic process [GO:0009450] Also known as: down regulation of 4-aminobutanoate catabolic process, down regulation of 4-aminobutanoate catabolism, down regulation of 4-aminobutyrate catabolic process, down regulation of 4-aminobutyrate catabolism, down regulation of GABA catabolic process, down regulation of GABA catabolism, down regulation of gamma-aminobutyric acid breakdown, down regulation of gamma-aminobutyric acid catabolic process, down regulation of gamma-aminobutyric acid catabolism, down regulation of gamma-aminobutyric acid degradation, down-regulation of 4-aminobutanoate catabolic process, down-regulation of 4-aminobutanoate catabolism, down-regulation of 4-aminobutyrate catabolic process, down-regulation of 4-aminobutyrate catabolism, down-regulation of GABA catabolic process, down-regulation of GABA catabolism, down-regulation of gamma-aminobutyric acid breakdown, down-regulation of gamma-aminobutyric acid catabolic process, down-regulation of gamma-aminobutyric acid catabolism, down-regulation of gamma-aminobutyric acid degradation, downregulation of 4-aminobutanoate catabolic process, downregulation of 4-aminobutanoate catabolism, downregulation of 4-aminobutyrate catabolic process, downregulation of 4-aminobutyrate catabolism, downregulation of GABA catabolic process, downregulation of GABA catabolism, downregulation of gamma-aminobutyric acid breakdown, downregulation of gamma-aminobutyric acid catabolic process, downregulation of gamma-aminobutyric acid catabolism, downregulation of gamma-aminobutyric acid degradation, inhibition of 4-aminobutanoate catabolic process, inhibition of 4-aminobutanoate catabolism, inhibition of 4-aminobutyrate catabolic process, inhibition of 4-aminobutyrate catabolism, inhibition of GABA catabolic process, inhibition of GABA catabolism, inhibition of gamma-aminobutyric acid breakdown, inhibition of gamma-aminobutyric acid catabolism, inhibition of gamma-aminobutyric acid degradation, negative regulation of 4-aminobutanoate catabolic process, negative regulation of 4-aminobutanoate catabolism, negative regulation of 4-aminobutyrate catabolic process, negative regulation of 4-aminobutyrate catabolism, negative regulation of GABA catabolic process, negative regulation of GABA catabolism, negative regulation of gamma-aminobutyric acid breakdown, negative regulation of gamma-aminobutyric acid catabolism, negative regulation of gamma-aminobutyric acid degradation, inhibition of gamma-aminobutyric acid catabolic process